{
  "gene_symbol": "SMARCD2",
  "gene_name": "SWI_SNF-related matrix-associated actin-dependent regulator of chromatin subfamily D member 2",
  "gene": "UniProtKB:Q92925",
  "term_id": "GO:0006357",
  "term_label": "regulation of transcription by RNA polymerase II"
}